{
  "gene_symbol": "GRIPAP1",
  "term_id": "GO:0098998",
  "gene": "UniProtKB:Q4V328",
  "gene_name": "GRIP1-associated protein 1",
  "term_label": "extrinsic component of postsynaptic early endosome membrane"
}